{
  "gene_symbol": "OR5B17",
  "gene": "UniProtKB:Q8NGF7",
  "term_id": "GO:0007608",
  "term_label": "sensory perception of smell",
  "gene_name": "Olfactory receptor 5B17"
}